{
  "gene_symbol": "CSNK2A1",
  "term_label": "nucleus",
  "gene": "UniProtKB:P68400",
  "gene_name": "Casein kinase II subunit alpha",
  "term_id": "GO:0005634"
}